regulation of amino acid export [GO:0080143] (biological process) References: PMID:20018597 Definition: Any process that modulates the frequency, rate or extent of amino acid export. Amino acid export is the directed movement of amino acids out of a cell or organelle. Relationships: is a type of regulation of amino acid transmembrane transport [GO:1903789]; regulates amino acid export across plasma membrane [GO:0032973]